{
  "gene_name": "Golgin subfamily A member 6-like protein 7",
  "gene": "UniProtKB:A0A1B0GV03",
  "term_label": "Unknown cellular component",
  "term_id": "UNKNOWN:0003",
  "gene_symbol": "GOLGA6L7"
}